ochratoxin A biosynthetic process [GO:1900818] (biological process) Definition: The chemical reactions and pathways resulting in the formation of ochratoxin A. Relationships: is a type of modified amino acid biosynthetic process [GO:0042398]; is a type of GO:0043604; is a type of secondary metabolite biosynthetic process [GO:0044550]; is a type of monocarboxylic acid biosynthetic process [GO:0072330]; is a type of organohalogen metabolic process [GO:0090345] Sources: GOC:TermGenie, GOC:di Also known as: Ochratoxin A anabolism, Ochratoxin A biosynthesis, Ochratoxin A formation, Ochratoxin A synthesis